{
  "gene": "UniProtKB:Q8WXK4",
  "term_id": "GO:0061630",
  "term_label": "ubiquitin protein ligase activity",
  "gene_symbol": "ASB12",
  "gene_name": "Ankyrin repeat and SOCS box protein 12"
}